lignin metabolic process [GO:0009808] (biological process) Relationships: is a type of phenylpropanoid metabolic process [GO:0009698] Sources: GOC:lr, GOC:yl Subtypes: lignin biosynthetic process [GO:0009809], GO:0046274 Also known as: lignin metabolism Definition: The chemical reactions and pathways involving lignins, a class of polymers of phenylpropanoid units.